{
  "term_label": "establishment of endothelial intestinal barrier",
  "gene_symbol": "TJP1",
  "gene_name": "Tight junction protein ZO-1",
  "gene": "UniProtKB:Q07157",
  "term_id": "GO:0090557"
}